{
  "term_label": "cytoplasmic vesicle",
  "term_id": "GO:0031410",
  "gene_name": "Flotillin-2",
  "gene": "UniProtKB:Q14254",
  "gene_symbol": "FLOT2"
}